{
  "gene": "UniProtKB:Q13118",
  "gene_name": "Krueppel-like factor 10",
  "gene_symbol": "KLF10",
  "term_id": "GO:0000978",
  "term_label": "RNA polymerase II cis-regulatory region sequence-specific DNA binding"
}